{
  "gene_symbol": "OR10H1",
  "gene": "UniProtKB:Q9Y4A9",
  "term_id": "GO:0005886",
  "term_label": "plasma membrane",
  "gene_name": "Olfactory receptor 10H1"
}